{
  "gene": "UniProtKB:O14810",
  "gene_symbol": "CPLX1",
  "term_label": "modulation of chemical synaptic transmission",
  "gene_name": "Complexin-1",
  "term_id": "GO:0050804"
}